{
  "gene_name": "Uncharacterized protein FLJ46757",
  "term_id": "UNKNOWN:0002",
  "gene_symbol": "Q6ZR03",
  "term_label": "Unknown biological process",
  "gene": "UniProtKB:Q6ZR03"
}